{
  "term_label": "damaged DNA binding",
  "gene_symbol": "RBBP8",
  "gene": "UniProtKB:Q99708",
  "gene_name": "DNA endonuclease RBBP8",
  "term_id": "GO:0003684"
}